{
  "term_id": "UNKNOWN:0002",
  "term_label": "Unknown biological process",
  "gene_name": "dTDP-D-glucose 4,6-dehydratase",
  "gene": "UniProtKB:O95455",
  "gene_symbol": "TGDS"
}